{
  "gene": "UniProtKB:Q9Y4H2",
  "term_id": "GO:0008286",
  "term_label": "insulin receptor signaling pathway",
  "gene_name": "Insulin receptor substrate 2",
  "gene_symbol": "IRS2"
}